{
  "gene_symbol": "YIPF2",
  "term_id": "GO:0005794",
  "gene": "UniProtKB:Q9BWQ6",
  "gene_name": "Protein YIPF2",
  "term_label": "Golgi apparatus"
}